{
  "gene_name": "Ras-related protein Rab-11B",
  "term_label": "Golgi apparatus",
  "term_id": "GO:0005794",
  "gene_symbol": "RAB11B",
  "gene": "UniProtKB:Q15907"
}